{
  "term_id": "GO:0045202",
  "term_label": "synapse",
  "gene_symbol": "CHRM1",
  "gene": "UniProtKB:P11229",
  "gene_name": "Muscarinic acetylcholine receptor M1"
}